tumor necrosis factor-mediated signaling pathway [GO:0033209] (BP) Sources: GOC:mah, GOC:signaling Regulation: regulated by regulation of tumor necrosis factor-mediated signaling pathway [GO:0010803]; negatively regulated by negative regulation of tumor necrosis factor-mediated signaling pathway [GO:0010804]; positively regulated by positive regulation of tumor necrosis factor-mediated signaling pathway [GO:1903265] Also known as: tumor necrosis factor-mediated signalling pathway, TNF-alpha-mediated signaling pathway, tumor necrosis factor alpha-mediated signaling pathway, adipocytokine signaling pathway Relationships: is a type of cytokine-mediated signaling pathway [GO:0019221]; is part of cellular response to tumor necrosis factor [GO:0071356] Definition: The series of molecular signals initiated by tumor necrosis factor binding to its receptor on the surface of a cell, and ending with the regulation of a downstream cellular process, e.g. transcription.